{
  "gene": "UniProtKB:Q15323",
  "term_label": "morphogenesis of an epithelium",
  "term_id": "GO:0002009",
  "gene_symbol": "KRT31",
  "gene_name": "Keratin, type I cuticular Ha1"
}